{
  "gene_symbol": "CRLF2",
  "term_label": "cytokine binding",
  "gene": "UniProtKB:Q9HC73",
  "gene_name": "Cytokine receptor-like factor 2",
  "term_id": "GO:0019955"
}